{
  "gene": "UniProtKB:Q2M2I3",
  "term_id": "UNKNOWN:0003",
  "gene_symbol": "FAM83E",
  "term_label": "Unknown cellular component",
  "gene_name": "Protein FAM83E"
}